CDP-abequose epimerase activity [GO:0047732] (molecular function) Sources: EC:5.1.3.10, RHEA:21656 Also known as: CDP-3,6-dideoxy-D-glucose 2-epimerase activity, CDP-D-abequose 2-epimerase activity, CDP-paratose 2-epimerase activity, CDP-paratose epimerase activity, CDP-tyvelose 2-epimerase activity, cytidine diphosphate paratose-2-epimerase activity, cytidine diphosphoabequose epimerase activity, cytidine diphosphodideoxyglucose epimerase activity, cytidine diphosphoparatose epimerase activity Definition: Catalysis of the reaction: CDP-3,6-dideoxy-D-glucose = CDP-3,6-dideoxy-D-mannose. Relationships: is a type of GO:0016857